{
  "term_label": "mRNA splicing, via spliceosome",
  "gene_symbol": "PLRG1",
  "gene_name": "Pleiotropic regulator 1",
  "term_id": "GO:0000398",
  "gene": "UniProtKB:O43660"
}